{
  "gene": "UniProtKB:Q9ULW6",
  "term_id": "GO:0005634",
  "gene_symbol": "NAP1L2",
  "term_label": "nucleus",
  "gene_name": "Nucleosome assembly protein 1-like 2"
}